{
  "term_id": "UNKNOWN:0001",
  "gene_symbol": "GOLM2",
  "term_label": "Unknown molecular function",
  "gene_name": "Protein GOLM2",
  "gene": "UniProtKB:Q6P4E1"
}